positive regulation of osteoclast differentiation [GO:0045672] (biological process) Also known as: up regulation of osteoclast differentiation, up-regulation of osteoclast differentiation, upregulation of osteoclast differentiation, activation of osteoclast differentiation, stimulation of osteoclast differentiation Definition: Any process that activates or increases the frequency, rate or extent of osteoclast differentiation. Subtypes: GO:2001206 Relationships: is a type of positive regulation of myeloid leukocyte differentiation [GO:0002763]; is a type of regulation of osteoclast differentiation [GO:0045670]; positively regulates osteoclast differentiation [GO:0030316] Sources: GOC:go_curators